D2 dopamine receptor binding [GO:0031749] (MF) Sources: GOC:mah, GOC:nln Relationships: is_a dopamine receptor binding [GO:0050780] Also known as: D2 dopamine receptor ligand Definition: Binding to a D2 dopamine receptor.